{
  "term_id": "GO:0002009",
  "gene_name": "Keratin, type I cytoskeletal 16",
  "gene_symbol": "KRT16",
  "gene": "UniProtKB:P08779",
  "term_label": "morphogenesis of an epithelium"
}